negative regulation of peptidyl-serine phosphorylation of STAT protein [GO:0033140] (biological process) Also known as: down regulation of serine phosphorylation of STAT3 protein, down-regulation of serine phosphorylation of STAT3 protein, downregulation of serine phosphorylation of STAT3 protein, inhibition of serine phosphorylation of STAT3 protein, negative regulation of serine phosphorylation of STAT3 protein Sources: GOC:mah Definition: Any process that stops, prevents, or reduces the frequency, rate or extent of the phosphorylation of a serine residue of a STAT (Signal Transducer and Activator of Transcription) protein. Relationships: is_a negative regulation of peptidyl-serine phosphorylation [GO:0033137]; is a type of regulation of peptidyl-serine phosphorylation of STAT protein [GO:0033139]; negatively regulates GO:0042501